pigmentation [GO:0043473] (biological process) Definition: The accumulation of pigment in an organism, tissue or cell, either by increased deposition or by increased number of cells. Sources: GOC:jl Subtypes: cellular pigmentation [GO:0033059], ocellus pigmentation [GO:0033060], pigment accumulation [GO:0043476], developmental pigmentation [GO:0048066] Relationships: is a type of biological_process [GO:0008150] Regulation: regulated by regulation of pigmentation [GO:0120305]